{
  "gene": "UniProtKB:Q8WXH0",
  "term_label": "nuclear migration",
  "term_id": "GO:0007097",
  "gene_name": "Nesprin-2",
  "gene_symbol": "SYNE2"
}